negative regulation of cardiac conduction [GO:1903780] (biological process) Relationships: is a type of negative regulation of biological process [GO:0048519]; is a type of GO:1903779; negatively regulates cardiac conduction [GO:0061337] Definition: Any process that stops, prevents or reduces the frequency, rate or extent of cardiac conduction. References: PMID:12967627 Sources: GOC:BHF, GOC:TermGenie, GOC:mtg_cardiac_conduct_nov11, GOC:rph, GO_REF:0000058 Also known as: down regulation of cardiac conduction, down-regulation of cardiac conduction, downregulation of cardiac conduction, inhibition of cardiac conduction